{
  "term_id": "UNKNOWN:0001",
  "gene": "UniProtKB:Q5T681",
  "term_label": "Unknown molecular function",
  "gene_name": "Uncharacterized protein C10orf62",
  "gene_symbol": "C10orf62"
}